{
  "gene_name": "3-ketoacyl-CoA thiolase, mitochondrial",
  "gene": "UniProtKB:P42765",
  "gene_symbol": "ACAA2",
  "term_id": "GO:0006635",
  "term_label": "fatty acid beta-oxidation"
}